{
  "gene_symbol": "GTF2F2",
  "term_id": "GO:0005674",
  "gene_name": "General transcription factor IIF subunit 2",
  "term_label": "transcription factor TFIIF complex",
  "gene": "UniProtKB:P13984"
}